{
  "term_label": "Unknown biological process",
  "term_id": "UNKNOWN:0002",
  "gene_symbol": "SMIM42",
  "gene_name": "Small integral membrane protein 42",
  "gene": "UniProtKB:A0A5F9ZH02"
}